{
  "gene": "UniProtKB:Q8TCJ2",
  "term_id": "GO:0004579",
  "gene_name": "Dolichyl-diphosphooligosaccharide--protein glycosyltransferase subunit STT3B",
  "term_label": "dolichyl-diphosphooligosaccharide-protein glycotransferase activity",
  "gene_symbol": "STT3B"
}